{
  "gene": "UniProtKB:Q02575",
  "gene_symbol": "NHLH1",
  "term_label": "RNA polymerase II cis-regulatory region sequence-specific DNA binding",
  "term_id": "GO:0000978",
  "gene_name": "Helix-loop-helix protein 1"
}